{
  "term_label": "receptor antagonist activity",
  "gene": "UniProtKB:Q8IVG9",
  "gene_symbol": "MT-RNR2",
  "term_id": "GO:0048019",
  "gene_name": "Humanin"
}